{
  "gene": "UniProtKB:O14933",
  "gene_name": "Ubiquitin_ISG15-conjugating enzyme E2 L6",
  "term_id": "GO:0005634",
  "term_label": "nucleus",
  "gene_symbol": "UBE2L6"
}